{
  "gene_symbol": "IFNA4",
  "gene": "UniProtKB:P05014",
  "term_id": "GO:0060337",
  "term_label": "type I interferon-mediated signaling pathway",
  "gene_name": "Interferon alpha-4"
}